{
  "gene_symbol": "CYP3A5",
  "term_id": "GO:0070989",
  "gene_name": "Cytochrome P450 3A5",
  "gene": "UniProtKB:P20815",
  "term_label": "oxidative demethylation"
}